{
  "gene": "UniProtKB:Q9NRY4",
  "gene_symbol": "ARHGAP35",
  "term_label": "regulation of cell size",
  "term_id": "GO:0008361",
  "gene_name": "Rho GTPase-activating protein 35"
}